{
  "gene": "UniProtKB:P0C617",
  "term_id": "UNKNOWN:0001",
  "gene_symbol": "OR5AL1",
  "gene_name": "Olfactory receptor 5AL1",
  "term_label": "Unknown molecular function"
}